{
  "term_label": "hyperosmotic response",
  "gene": "UniProtKB:P29972",
  "term_id": "GO:0006972",
  "gene_name": "Aquaporin-1",
  "gene_symbol": "AQP1"
}